{
  "term_label": "regulation of transcription by RNA polymerase II",
  "gene_name": "Zinc finger protein 596",
  "term_id": "GO:0006357",
  "gene_symbol": "ZNF596",
  "gene": "UniProtKB:Q8TC21"
}